{
  "gene": "UniProtKB:O95816",
  "term_label": "protein stabilization",
  "gene_symbol": "BAG2",
  "term_id": "GO:0050821",
  "gene_name": "BAG family molecular chaperone regulator 2"
}